metaphase plate [GO:0070090] (CC) Relationships: is_a intracellular anatomical structure [GO:0005622] Definition: The intracellular plane, located halfway between the poles of the spindle, where chromosomes align during metaphase of mitotic or meiotic nuclear division. Sources: GOC:mah